{
  "term_label": "transcription factor TFIID complex",
  "gene": "UniProtKB:P21675",
  "gene_symbol": "TAF1",
  "term_id": "GO:0005669",
  "gene_name": "Transcription initiation factor TFIID subunit 1"
}